{
  "gene_symbol": "TMEM259",
  "term_id": "UNKNOWN:0001",
  "gene_name": "Membralin",
  "term_label": "Unknown molecular function",
  "gene": "UniProtKB:Q4ZIN3"
}